regulation of oligodendrocyte differentiation [GO:0048713] (biological process) Subtypes: GO:0048714, negative regulation of oligodendrocyte differentiation [GO:0048715] Relationships: is a type of regulation of glial cell differentiation [GO:0045685]; regulates oligodendrocyte differentiation [GO:0048709] References: PMID:15139015 Sources: GOC:vp Definition: Any process that modulates the frequency, rate or extent of oligodendrocyte differentiation.